{
  "gene_name": "Transcriptional repressor CTCF",
  "gene": "UniProtKB:P49711",
  "gene_symbol": "CTCF",
  "term_id": "GO:0006357",
  "term_label": "regulation of transcription by RNA polymerase II"
}